{
  "gene": "UniProtKB:O94986",
  "gene_name": "Centrosomal protein of 152 kDa",
  "term_label": "Unknown molecular function",
  "gene_symbol": "CEP152",
  "term_id": "UNKNOWN:0001"
}